mastigoneme [GO:0097741] (cellular component) Relationships: is a type of GO:0099080; is part of motile cilium [GO:0031514] Definition: A hair-like structure covering the flagella found in some algae (heterokonts and cryptophytes). It is approximately 15 nm in diameter, and usually consist of a tubular shaft that itself terminates in smaller hairs. It is composed of glycoproteins and, likely, carbohydrates. Mastigonemes may assist in locomotion by increasing the surface area of a flagellum. References: PMID:943397 Sources: GOC:cilia, Wikipedia:Mastigoneme